negative regulation of immature T cell proliferation in thymus [GO:0033088] (biological process) Definition: Any process that stops, prevents, or reduces the frequency, rate or extent of immature T cell proliferation in the thymus. Sources: GOC:add, GOC:mah Relationships: is a type of regulation of immature T cell proliferation in thymus [GO:0033084]; is_a negative regulation of T cell differentiation in thymus [GO:0033085]; is a type of negative regulation of immature T cell proliferation [GO:0033087]; negatively regulates immature T cell proliferation in thymus [GO:0033080] Also known as: negative regulation of thymic T cell proliferation, negative regulation of thymocyte cell proliferation, negative regulation of thymocyte proliferation